{
  "gene_name": "Bombesin receptor-activated protein C6orf89",
  "gene": "UniProtKB:Q6UWU4",
  "term_label": "Unknown molecular function",
  "term_id": "UNKNOWN:0001",
  "gene_symbol": "C6orf89"
}